{
  "gene_symbol": "PLCL1",
  "gene_name": "Inactive phospholipase C-like protein 1",
  "gene": "UniProtKB:Q15111",
  "term_id": "GO:0048015",
  "term_label": "phosphatidylinositol-mediated signaling"
}